{
  "term_label": "syntaxin-1 binding",
  "gene": "UniProtKB:P63027",
  "gene_symbol": "VAMP2",
  "gene_name": "Vesicle-associated membrane protein 2",
  "term_id": "GO:0017075"
}